{
  "gene_symbol": "CRYBG2",
  "term_id": "UNKNOWN:0001",
  "term_label": "Unknown molecular function",
  "gene_name": "Beta_gamma crystallin domain-containing protein 2",
  "gene": "UniProtKB:Q8N1P7"
}